{
  "gene_name": "PITH domain-containing protein 1",
  "gene": "UniProtKB:Q9GZP4",
  "gene_symbol": "PITHD1",
  "term_label": "Unknown biological process",
  "term_id": "UNKNOWN:0002"
}